{
  "gene": "UniProtKB:P55285",
  "gene_name": "Cadherin-6",
  "term_label": "catenin complex",
  "term_id": "GO:0016342",
  "gene_symbol": "CDH6"
}